{
  "gene": "UniProtKB:O75509",
  "gene_symbol": "TNFRSF21",
  "term_label": "oligodendrocyte apoptotic process",
  "term_id": "GO:0097252",
  "gene_name": "Tumor necrosis factor receptor superfamily member 21"
}